spindle assembly involved in male meiosis I [GO:0007054] (biological process) Sources: GOC:mah Also known as: male meiosis I spindle assembly Definition: The formation of the spindle during meiosis I of a meiotic cell cycle in males. An example of this is found in Drosophila melanogaster. Relationships: is a type of spindle assembly involved in male meiosis [GO:0007053]; is part of male meiosis I [GO:0007141]